{
  "term_id": "GO:0005615",
  "gene_symbol": "FGG",
  "gene_name": "Fibrinogen gamma chain",
  "gene": "UniProtKB:P02679",
  "term_label": "extracellular space"
}